{
  "gene": "UniProtKB:H3BR10",
  "term_id": "UNKNOWN:0002",
  "gene_symbol": "SMLR1",
  "gene_name": "Small leucine-rich protein 1",
  "term_label": "Unknown biological process"
}